{
  "gene_symbol": "MBD2",
  "gene": "UniProtKB:Q9UBB5",
  "gene_name": "Methyl-CpG-binding domain protein 2",
  "term_id": "GO:0000122",
  "term_label": "negative regulation of transcription by RNA polymerase II"
}